neuroblast activation [GO:0007407] (biological process) Definition: A change in the morphology or behavior of a neuroblast resulting from exposure to an activating factor such as a cellular or soluble ligand. Sources: GOC:go_curators, GOC:mtg_sensu Relationships: is a type of cell activation [GO:0001775]; is part of GO:0048699